maltoheptaose metabolic process [GO:2001122] (biological process) Definition: The chemical reactions and pathways involving a maltoheptaose. Sources: GOC:mengo_curators Relationships: is a type of GO:0009311 Subtypes: GO:2001123 Also known as: maltoheptaose metabolism